{
  "gene_name": "Transcription factor 20",
  "gene_symbol": "TCF20",
  "gene": "UniProtKB:Q9UGU0",
  "term_id": "GO:0003713",
  "term_label": "transcription coactivator activity"
}